{
  "gene": "UniProtKB:Q765P7",
  "term_label": "phospholipid binding",
  "term_id": "GO:0005543",
  "gene_name": "Protein MTSS 2",
  "gene_symbol": "MTSS2"
}